{
  "term_id": "GO:0010887",
  "gene": "UniProtKB:Q07869",
  "gene_name": "Peroxisome proliferator-activated receptor alpha",
  "term_label": "negative regulation of cholesterol storage",
  "gene_symbol": "PPARA"
}